regulation of semaphorin-plexin signaling pathway [GO:2001260] (BP) Definition: Any process that modulates the frequency, rate or extent of semaphorin-plexin signaling pathway. Subtypes: negative regulation of semaphorin-plexin signaling pathway [GO:2001261], positive regulation of semaphorin-plexin signaling pathway [GO:2001262] Also known as: regulation of semaphorin-plexin signalling pathway Sources: GOC:BHF Relationships: is a type of regulation of signal transduction [GO:0009966]; regulates semaphorin-plexin signaling pathway [GO:0071526]